{
  "gene": "UniProtKB:A1A519",
  "gene_name": "Protein FAM170A",
  "term_label": "Unknown molecular function",
  "gene_symbol": "FAM170A",
  "term_id": "UNKNOWN:0001"
}